{
  "gene_name": "Septin-1",
  "term_id": "GO:0032153",
  "term_label": "cell division site",
  "gene_symbol": "SEPTIN1",
  "gene": "UniProtKB:Q8WYJ6"
}